{
  "term_label": "protein serine/threonine kinase activator activity",
  "gene_name": "T-cell leukemia_lymphoma protein 1A",
  "term_id": "GO:0043539",
  "gene": "UniProtKB:P56279",
  "gene_symbol": "TCL1A"
}